{
  "term_label": "plasma membrane",
  "term_id": "GO:0005886",
  "gene_symbol": "GPR176",
  "gene": "UniProtKB:Q14439",
  "gene_name": "G-protein coupled receptor 176"
}